{
  "term_label": "cytoplasm",
  "term_id": "GO:0005737",
  "gene_symbol": "SPOP",
  "gene_name": "Speckle-type POZ protein",
  "gene": "UniProtKB:O43791"
}